{
  "term_label": "septin complex",
  "gene": "UniProtKB:Q16181",
  "gene_name": "Septin-7",
  "gene_symbol": "SEPTIN7",
  "term_id": "GO:0031105"
}